{
  "gene_name": "Putative transmembrane protein encoded by LINC00862",
  "gene": "UniProtKB:A6NCI5",
  "gene_symbol": "LINC00862",
  "term_label": "Unknown molecular function",
  "term_id": "UNKNOWN:0001"
}